perinucleolar compartment [GO:0097356] (cellular component) Relationships: is a type of cellular anatomical structure [GO:0110165]; is part of nuclear lumen [GO:0031981] References: PMID:21385875 Sources: GOC:vw, Wikipedia:Perinucleolar_compartment Also known as: perinucleolar region Definition: The perinucleolar compartment (PNC) is a subnuclear structure associated with, but structurally distinct from, the nucleolus. The PNC contains large amounts of the heterogeneous nuclear ribonucleoprotein complex (hnRNP) called hnRNP 1 (PTB). Many RNA binding proteins as well as RNA polymerase III transcripts are highly enriched in this compartment. PTB and pol III transcripts are required for the integrity of the PNC.